{
  "gene_symbol": "ZNF227",
  "term_id": "GO:0006357",
  "gene": "UniProtKB:Q86WZ6",
  "gene_name": "Zinc finger protein 227",
  "term_label": "regulation of transcription by RNA polymerase II"
}